positive regulation of cell proliferation in dorsal spinal cord [GO:1902833] (biological process) References: PMID:21730158 Sources: GOC:TermGenie, GOC:mr, GO_REF:0000058 Definition: Any process that activates or increases the frequency, rate or extent of cell proliferation in dorsal spinal cord. Also known as: up regulation of cell proliferation in dorsal spinal cord, up-regulation of cell proliferation in dorsal spinal cord, upregulation of cell proliferation in dorsal spinal cord, activation of cell proliferation in dorsal spinal cord Relationships: is a type of regulation of cell proliferation in dorsal spinal cord [GO:0021921]; is a type of positive regulation of neural precursor cell proliferation [GO:2000179]; positively regulates cell proliferation in dorsal spinal cord [GO:0010456]